{
  "gene": "UniProtKB:O14842",
  "term_label": "response to fatty acid",
  "gene_name": "Free fatty acid receptor 1",
  "term_id": "GO:0070542",
  "gene_symbol": "FFAR1"
}